{
  "term_id": "GO:0035686",
  "gene_name": "Sperm surface protein Sp17",
  "gene_symbol": "SPA17",
  "term_label": "sperm fibrous sheath",
  "gene": "UniProtKB:Q15506"
}